{
  "gene_symbol": "GYS1",
  "gene": "UniProtKB:P13807",
  "gene_name": "Glycogen [starch] synthase, muscle",
  "term_id": "GO:0005737",
  "term_label": "cytoplasm"
}